scintillon [GO:0036007] (cellular component) Definition: A body present in the cytoplasm of some dinoflagellates, which is the source of bioluminescence; emits light on acidification in the presence of oxygen. Relationships: is a type of cellular anatomical structure [GO:0110165]; is part of cytoplasm [GO:0005737] References: PMID:4501583, PMID:5642469 Sources: GOC:mag, GOC:pr